negative regulation of Schwann cell differentiation [GO:0014039] (biological process) Definition: Any process that stops, prevents, or reduces the frequency, rate or extent of Schwann cell differentiation. Also known as: down regulation of Schwann cell differentiation, down-regulation of Schwann cell differentiation, downregulation of Schwann cell differentiation, inhibition of Schwann cell differentiation Sources: GOC:ef Relationships: is a type of regulation of Schwann cell differentiation [GO:0014038]; is a type of GO:0045686; negatively regulates Schwann cell differentiation [GO:0014037]